meprin A complex [GO:0017090] (cellular component) Also known as: PABA peptide hydrolase complex Relationships: is a type of GO:0098796 Sources: GOC:mah, MEROPS_fam:M12 Definition: A protein complex that is located in the cell membrane, and is involved in the metabolism of peptides, including neuropeptides. The complex has metalloendopeptidase activity that catalyzes the hydrolysis of protein and peptide substrates, preferentially on carboxyl side of hydrophobic residues.